{
  "gene": "UniProtKB:P43657",
  "gene_symbol": "LPAR6",
  "gene_name": "Lysophosphatidic acid receptor 6",
  "term_label": "lysophosphatidic acid receptor activity",
  "term_id": "GO:0070915"
}